{
  "term_id": "UNKNOWN:0001",
  "term_label": "Unknown molecular function",
  "gene_name": "Minichromosome maintenance domain-containing protein 2",
  "gene": "UniProtKB:Q4G0Z9",
  "gene_symbol": "MCMDC2"
}